{
  "gene_symbol": "PKD2",
  "gene_name": "Polycystin-2",
  "term_label": "calcium ion binding",
  "gene": "UniProtKB:Q13563",
  "term_id": "GO:0005509"
}